{
  "gene_symbol": "GCNA",
  "gene_name": "Germ cell nuclear acidic protein",
  "term_label": "nucleus",
  "gene": "UniProtKB:Q96QF7",
  "term_id": "GO:0005634"
}